{
  "gene": "UniProtKB:O43677",
  "gene_symbol": "NDUFC1",
  "gene_name": "NADH dehydrogenase [ubiquinone] 1 subunit C1, mitochondrial",
  "term_label": "Unknown molecular function",
  "term_id": "UNKNOWN:0001"
}